behavioral response to starvation [GO:0042595] (biological process) Also known as: behavioural response to starvation Sources: GOC:go_curators Definition: Any process that results in a change in the behavior of an organism as a result of deprivation of nourishment. Relationships: is a type of GO:0042594